{
  "gene": "UniProtKB:Q9UQB3",
  "term_id": "GO:0005737",
  "gene_symbol": "CTNND2",
  "term_label": "cytoplasm",
  "gene_name": "Catenin delta-2"
}